aerobic respiration, using nitrite as electron donor [GO:0019332] (biological process) Definition: The oxidation of nitrite (NO2) to nitrate (NO3), using oxygen (O2) as the electron acceptor. Nitrite oxidation is the final step in nitrification, the oxidation of ammonia to nitrate, and nitrite oxidoreductase (NOR) is the key enzyme complex that catalyzes the conversion of nitrite to nitrate in nitrite oxidizing species. Sources: MetaCyc:P282-PWY Relationships: is a type of aerobic respiration [GO:0009060]; is a type of energy derivation by oxidation of reduced inorganic compounds [GO:0015975] Also known as: nitrite oxidation